regulation of sorocarp spore cell differentiation [GO:1901261] (biological process) Definition: Any process that modulates the frequency, rate or extent of sorocarp spore cell differentiation. Sources: GOC:TermGenie, GOC:rjd Relationships: is a type of regulation of sorocarp development [GO:0031156]; is a type of regulation of cell differentiation [GO:0045595]; regulates sorocarp spore cell differentiation [GO:0044671] Subtypes: cheating during chimeric sorocarp development [GO:0099139], negative regulation of sorocarp spore cell differentiation [GO:1901262], GO:1901263